{
  "gene": "UniProtKB:Q6ZN28",
  "gene_name": "Metastasis-associated in colon cancer protein 1",
  "term_label": "Unknown biological process",
  "term_id": "UNKNOWN:0002",
  "gene_symbol": "MACC1"
}